{
  "gene_symbol": "IFNB1",
  "term_id": "GO:0043330",
  "gene_name": "Interferon beta",
  "gene": "UniProtKB:P01574",
  "term_label": "response to exogenous dsRNA"
}